{
  "gene_name": "Golgin subfamily A member 6B",
  "term_label": "Golgi organization",
  "term_id": "GO:0007030",
  "gene": "UniProtKB:A6NDN3",
  "gene_symbol": "GOLGA6B"
}